{
  "term_label": "cytoskeleton-dependent cytokinesis",
  "gene_symbol": "SEPTIN9",
  "gene": "UniProtKB:Q9UHD8",
  "gene_name": "Septin-9",
  "term_id": "GO:0061640"
}